{
  "gene_symbol": "PLA2G4F",
  "gene": "UniProtKB:Q68DD2",
  "gene_name": "Cytosolic phospholipase A2 zeta",
  "term_id": "GO:0005544",
  "term_label": "calcium-dependent phospholipid binding"
}